{
  "gene": "UniProtKB:Q8IYJ3",
  "gene_symbol": "SYTL1",
  "term_label": "exocytosis",
  "gene_name": "Synaptotagmin-like protein 1",
  "term_id": "GO:0006887"
}